{
  "gene_name": "DNA topoisomerase 3-beta-1",
  "gene_symbol": "TOP3B",
  "gene": "UniProtKB:O95985",
  "term_id": "GO:0003917",
  "term_label": "DNA topoisomerase type I (single strand cut, ATP-independent) activity"
}